{
  "term_id": "GO:0005220",
  "gene_name": "Inositol 1,4,5-trisphosphate receptor type 3",
  "gene": "UniProtKB:Q14573",
  "gene_symbol": "ITPR3",
  "term_label": "inositol 1,4,5-trisphosphate-gated calcium channel activity"
}